5,6-dihydroxy-3-methyl-2-oxo-1,2,5,6-tetrahydroquinoline dehydrogenase activity [GO:0018518] (molecular function) Relationships: is a type of oxidoreductase activity, acting on the CH-CH group of donors, NAD or NADP as acceptor [GO:0016628] Definition: Catalysis of the reaction: 5,6-dihydroxy-3-methyl-5,6-dihydroquinolin-2(1H)-one + NAD+ = 5,6-dihydroxy-3-methyl-2-oxo-1,2-dihydroquinoline + H+ + NADH. Also known as: 5,6-dihydrodiol-3-methyl-2-oxo-1,2-dihydroquinoline dehydrogenase, 5,6-dihydroxy-3-methyl-2-oxo-1,2,5,6-tetrahydroquinoline:NAD+ oxidoreductase activity Sources: EC:1.3.1.65, RHEA:24556